{
  "term_label": "brain development",
  "gene": "UniProtKB:O75298",
  "gene_symbol": "RTN2",
  "gene_name": "Reticulon-2",
  "term_id": "GO:0007420"
}